{
  "term_id": "GO:0005112",
  "term_label": "Notch binding",
  "gene": "UniProtKB:Q6UY11",
  "gene_symbol": "DLK2",
  "gene_name": "Protein delta homolog 2"
}